{
  "term_label": "Unknown biological process",
  "gene_name": "GMP reductase 1",
  "gene_symbol": "GMPR",
  "gene": "UniProtKB:P36959",
  "term_id": "UNKNOWN:0002"
}